negative regulation of NF-kappaB transcription factor activity [GO:0032088] (biological process) Also known as: inhibition of NF-kappaB transcription factor, NF-kappaB inhibitor Relationships: is_a negative regulation of DNA-binding transcription factor activity [GO:0043433] Definition: Any process that stops, prevents, or reduces the frequency, rate or extent of the activity of the transcription factor NF-kappaB. Sources: GOC:dph, GOC:rl, GOC:tb